{
  "term_id": "GO:0005739",
  "gene_name": "Large ribosomal subunit protein bL35m",
  "term_label": "mitochondrion",
  "gene_symbol": "MRPL35",
  "gene": "UniProtKB:Q9NZE8"
}